{
  "term_id": "GO:0005736",
  "gene_symbol": "POLR1B",
  "gene_name": "DNA-directed RNA polymerase I subunit RPA2",
  "gene": "UniProtKB:Q9H9Y6",
  "term_label": "RNA polymerase I complex"
}